{
  "gene": "UniProtKB:Q7Z6J6",
  "term_label": "Unknown molecular function",
  "term_id": "UNKNOWN:0001",
  "gene_name": "FERM domain-containing protein 5",
  "gene_symbol": "FRMD5"
}